{
  "term_label": "chloride channel activity",
  "gene_symbol": "GABRA6",
  "gene": "UniProtKB:Q16445",
  "term_id": "GO:0005254",
  "gene_name": "Gamma-aminobutyric acid receptor subunit alpha-6"
}